regulation of retinal ganglion cell axon guidance [GO:0090259] (biological process) Sources: GOC:tb, GOC:yaf Subtypes: GO:0090260, positive regulation of retinal ganglion cell axon guidance [GO:1902336] Definition: Any process that modulates the frequency, rate, or extent of retinal ganglion cell axon guidance, the process in which the migration of an axon growth cone of a retinal ganglion cell (RGC) is directed to its target in the brain in response to a combination of attractive and repulsive cues. Relationships: is a type of regulation of axon guidance [GO:1902667]; regulates retinal ganglion cell axon guidance [GO:0031290]